{
  "term_id": "GO:0017056",
  "gene": "UniProtKB:Q5SRE5",
  "gene_symbol": "NUP188",
  "term_label": "structural constituent of nuclear pore",
  "gene_name": "Nucleoporin NUP188"
}